{
  "gene_symbol": "POTEI",
  "term_id": "GO:0007409",
  "gene": "UniProtKB:P0CG38",
  "gene_name": "POTE ankyrin domain family member I",
  "term_label": "axonogenesis"
}